{
  "gene_symbol": "IL26",
  "term_label": "positive regulation of receptor signaling pathway via JAK-STAT",
  "term_id": "GO:0046427",
  "gene_name": "Interleukin-26",
  "gene": "UniProtKB:Q9NPH9"
}